RNA polymerase I transcription regulator complex [GO:0000120] (cellular component) Definition: A transcription factor complex that acts at a regulatory region of a gene transcribed by RNA polymerase I. Sources: GOC:mah Also known as: RNA polymerase I transcription factor complex Relationships: is a type of transcription regulator complex [GO:0005667]; is a type of GO:0140513; is part of nucleolus [GO:0005730] Subtypes: GO:0000500, GO:0005668, RNA polymerase I core factor complex [GO:0070860]